{
  "gene_symbol": "CCN6",
  "term_id": "GO:0031012",
  "gene": "UniProtKB:O95389",
  "gene_name": "Cellular communication network factor 6",
  "term_label": "extracellular matrix"
}